{
  "term_id": "GO:0005227",
  "gene_name": "Anoctamin-10",
  "gene_symbol": "ANO10",
  "term_label": "calcium-activated cation channel activity",
  "gene": "UniProtKB:Q9NW15"
}